{
  "gene_name": "Probable inactive tRNA-specific adenosine deaminase-like protein 3",
  "term_label": "cytoplasm",
  "gene": "UniProtKB:Q96EY9",
  "gene_symbol": "ADAT3",
  "term_id": "GO:0005737"
}